{
  "gene_name": "G patch domain-containing protein 4",
  "term_id": "UNKNOWN:0001",
  "term_label": "Unknown molecular function",
  "gene": "UniProtKB:Q5T3I0",
  "gene_symbol": "GPATCH4"
}